{
  "term_label": "extracellular space",
  "gene": "UniProtKB:P09683",
  "term_id": "GO:0005615",
  "gene_name": "Secretin",
  "gene_symbol": "SCT"
}